{
  "gene": "UniProtKB:Q9H205",
  "gene_name": "Olfactory receptor 2AG1",
  "term_id": "GO:0004984",
  "gene_symbol": "OR2AG1",
  "term_label": "olfactory receptor activity"
}